{
  "term_id": "GO:0048812",
  "term_label": "neuron projection morphogenesis",
  "gene_name": "Growth arrest-specific protein 7",
  "gene": "UniProtKB:O60861",
  "gene_symbol": "GAS7"
}